dGMP salvage [GO:0106384] (biological process) Definition: Any process which produces a dGMP from derivatives of it, without de novo synthesis. Relationships: is a type of dGMP biosynthetic process [GO:0006181]; is a type of purine deoxyribonucleotide salvage [GO:0106381] References: PMID:21829339, PMID:6605343